{
  "gene_name": "Adenine phosphoribosyltransferase",
  "gene": "UniProtKB:P07741",
  "gene_symbol": "APRT",
  "term_label": "adenine salvage",
  "term_id": "GO:0006168"
}